{
  "gene": "UniProtKB:Q9H0E7",
  "term_label": "regulation of cell cycle process",
  "gene_symbol": "USP44",
  "term_id": "GO:0010564",
  "gene_name": "Ubiquitin carboxyl-terminal hydrolase 44"
}